{
  "term_id": "GO:0097186",
  "gene_symbol": "ENAM",
  "gene": "UniProtKB:Q9NRM1",
  "term_label": "amelogenesis",
  "gene_name": "Enamelin"
}